{
  "term_label": "regulation of transcription by RNA polymerase II",
  "term_id": "GO:0006357",
  "gene": "UniProtKB:A9YTQ3",
  "gene_name": "Aryl hydrocarbon receptor repressor",
  "gene_symbol": "AHRR"
}